regulation of myofibril size [GO:0014881] (biological process) Relationships: is a type of GO:0014743; is a type of regulation of cellular component size [GO:0032535] Also known as: change of myofibril size Sources: GOC:dph, GOC:ef, GOC:mtg_muscle, GOC:tb Definition: Any process that modulates the size of myofibrils. A myofibril is the contractile element of skeletal and cardiac muscle. It is a long, highly organized bundle of actin, myosin, and other proteins that contracts by a sliding filament mechanism.